negative regulation of gliotoxin biosynthetic process [GO:1900690] (biological process) Also known as: down regulation of gliotoxin anabolism, down regulation of gliotoxin biosynthesis, down regulation of gliotoxin biosynthetic process, down regulation of gliotoxin formation, down regulation of gliotoxin synthesis, down-regulation of gliotoxin anabolism, down-regulation of gliotoxin biosynthesis, down-regulation of gliotoxin biosynthetic process, down-regulation of gliotoxin formation, down-regulation of gliotoxin synthesis, downregulation of gliotoxin anabolism, downregulation of gliotoxin biosynthesis, downregulation of gliotoxin biosynthetic process, downregulation of gliotoxin formation, downregulation of gliotoxin synthesis, inhibition of gliotoxin anabolism, inhibition of gliotoxin biosynthesis, inhibition of gliotoxin formation, inhibition of gliotoxin synthesis, negative regulation of gliotoxin anabolism, negative regulation of gliotoxin biosynthesis, negative regulation of gliotoxin formation, negative regulation of gliotoxin synthesis, inhibition of gliotoxin biosynthetic process Relationships: is a type of negative regulation of amide metabolic process [GO:0034249]; is a type of negative regulation of secondary metabolite biosynthetic process [GO:1900377]; is a type of regulation of gliotoxin biosynthetic process [GO:1900689]; negatively regulates gliotoxin biosynthetic process [GO:2001310] Sources: GOC:TermGenie, GOC:di Definition: Any process that stops, prevents or reduces the frequency, rate or extent of gliotoxin biosynthetic process.